regulation of Kit signaling pathway [GO:1900234] (biological process) Definition: Any process that modulates the frequency, rate or extent of Kit signaling pathway. Sources: GOC:TermGenie, GOC:signaling Subtypes: negative regulation of Kit signaling pathway [GO:1900235], positive regulation of Kit signaling pathway [GO:1900236] Relationships: is a type of GO:0001959; regulates GO:0038109 Also known as: regulation of Kit signalling pathway, regulation of stem cell factor receptor signaling pathway, regulation of stem cell factor signaling pathway